single-species submerged biofilm formation [GO:0090609] (biological process) Definition: A process in which planktonically growing microorganisms of the same species aggregate and grow on solid substrates under the flow of a liquid and produce extracellular polymers that facilitate attachment and matrix formation, resulting in a change in the organisms' growth rate and gene transcription. Sources: GOC:di, GOC:tb Relationships: is a type of GO:0044010; is_a GO:0090605 Subtypes: single-species biofilm formation on inanimate substrate [GO:0044011]